{
  "gene_name": "Zyxin",
  "term_label": "stress fiber",
  "gene_symbol": "ZYX",
  "term_id": "GO:0001725",
  "gene": "UniProtKB:Q15942"
}